{
  "term_label": "plasma membrane proton-transporting V-type ATPase complex",
  "gene": "UniProtKB:P61421",
  "gene_symbol": "ATP6V0D1",
  "term_id": "GO:0033181",
  "gene_name": "V-type proton ATPase subunit d 1"
}